{
  "gene_symbol": "LRRC8C",
  "term_id": "GO:0005886",
  "gene": "UniProtKB:Q8TDW0",
  "gene_name": "Volume-regulated anion channel subunit LRRC8C",
  "term_label": "plasma membrane"
}